{
  "gene": "UniProtKB:Q86T29",
  "gene_name": "Zinc finger protein 605",
  "term_id": "UNKNOWN:0003",
  "term_label": "Unknown cellular component",
  "gene_symbol": "ZNF605"
}